{
  "gene_symbol": "MAGEB18",
  "gene_name": "Melanoma-associated antigen B18",
  "gene": "UniProtKB:Q96M61",
  "term_label": "negative regulation of transcription by RNA polymerase II",
  "term_id": "GO:0000122"
}